{
  "term_id": "UNKNOWN:0002",
  "gene_name": "Ubiquitin carboxyl-terminal hydrolase 6",
  "term_label": "Unknown biological process",
  "gene_symbol": "USP6",
  "gene": "UniProtKB:P35125"
}